{
  "gene_symbol": "PDCD1LG2",
  "term_id": "GO:0007166",
  "term_label": "cell surface receptor signaling pathway",
  "gene": "UniProtKB:Q9BQ51",
  "gene_name": "Programmed cell death 1 ligand 2"
}